{
  "gene": "UniProtKB:P28222",
  "term_label": "chemical synaptic transmission",
  "term_id": "GO:0007268",
  "gene_name": "5-hydroxytryptamine receptor 1B",
  "gene_symbol": "HTR1B"
}